AP-4 adaptor complex [GO:0030124] (cellular component) Definition: An AP-type membrane coat adaptor complex that consists of beta4, epsilon, mu4 and sigma4 subunits and is found associated with membranes in the trans-Golgi network; it is not clear whether AP-4 forms clathrin coats in vivo. References: PMID:10611976 Sources: GOC:mah Relationships: is a type of AP-type membrane coat adaptor complex [GO:0030119]